{
  "gene_symbol": "PCNX3",
  "term_label": "Unknown molecular function",
  "gene": "UniProtKB:Q9H6A9",
  "term_id": "UNKNOWN:0001",
  "gene_name": "Pecanex-like protein 3"
}